ecdysis-triggering hormone receptor activity [GO:0042654] (molecular function) Relationships: is a type of GO:0004930; has part hormone binding [GO:0042562] Sources: GOC:ma Definition: Combining with ecdysis-triggering hormone to initiate a change in cell activity. Also known as: ETH receptor, ecdysis-triggering hormone binding